{
  "gene": "UniProtKB:A0A087WZ39",
  "gene_name": "T cell receptor beta variable 15 (Fragment)",
  "gene_symbol": "TRBV15",
  "term_id": "GO:0005886",
  "term_label": "plasma membrane"
}